NAD+-protein-serine ADP-ribosyltransferase activity [GO:0140805] (molecular function) Definition: Catalysis of the reaction: L-seryl-[protein] + NAD+ = H+ + nicotinamide + O-(ADP-D-ribosyl)-L-seryl-[protein]. References: PMID:32028527, PMID:33186521 Sources: RHEA:58232 Relationships: is a type of GO:1990404 Subtypes: GO:0140816, NAD+-histone H3S10 serine ADP-ribosyltransferase activity [GO:0140817]